{
  "term_id": "UNKNOWN:0001",
  "gene_symbol": "A6NN06",
  "term_label": "Unknown molecular function",
  "gene_name": "Putative UPF0633 protein MGC21881",
  "gene": "UniProtKB:A6NN06"
}